{
  "term_label": "protein serine/threonine kinase activity",
  "term_id": "GO:0004674",
  "gene_symbol": "ERN2",
  "gene_name": "Serine_threonine-protein kinase_endoribonuclease IRE2",
  "gene": "UniProtKB:Q76MJ5"
}